granum assembly [GO:0090391] (biological process) Sources: GOC:tb Definition: A process that is carried out at the cellular level which results in the assembly of a granum. A granum is a distinct stack of lamellae seen within chloroplasts. Relationships: is a type of cellular component assembly [GO:0022607]; is part of chloroplast organization [GO:0009658] Also known as: grana formation